{
  "gene_symbol": "MRGBP",
  "term_id": "UNKNOWN:0001",
  "term_label": "Unknown molecular function",
  "gene": "UniProtKB:Q9NV56",
  "gene_name": "MRG_MORF4L-binding protein"
}